{
  "gene_name": "Kelch repeat and BTB domain-containing protein 2",
  "term_label": "Cul3-RING ubiquitin ligase complex",
  "gene": "UniProtKB:Q8IY47",
  "term_id": "GO:0031463",
  "gene_symbol": "KBTBD2"
}